regulation of 1-aminocyclopropane-1-carboxylate metabolic process [GO:0010602] (biological process) Relationships: is a type of regulation of amino acid metabolic process [GO:0006521]; is a type of GO:0062012; regulates 1-aminocyclopropane-1-carboxylate metabolic process [GO:0018871] References: PMID:18055613 Definition: Regulation of the chemical reactions and pathways involving 1-aminocyclopropane-1-carboxylate, the anion of 1-aminocyclopropane-1-carboxylic acid, a natural product found in plant tissues. It is a key intermediate in the biosynthesis of ethylene (ethene), a fruit-ripening hormone in plants.